{
  "gene_symbol": "NAXD",
  "gene_name": "ATP-dependent (S)-NAD(P)H-hydrate dehydratase",
  "gene": "UniProtKB:Q8IW45",
  "term_label": "metabolite repair",
  "term_id": "GO:0110051"
}